regulation of cardiac muscle contraction by calcium ion signaling [GO:0010882] (biological process) Relationships: is a type of calcium-mediated signaling [GO:0019722]; is a type of GO:0055117 Subtypes: GO:0010881 Definition: Any process that modulates the frequency, rate or extent of cardiac muscle contraction by changing the calcium ion signals that trigger contraction. Sources: GOC:BHF, GOC:dph, GOC:tb Also known as: regulation of cardiac muscle contraction by calcium ion signalling